{
  "term_id": "GO:0005525",
  "term_label": "GTP binding",
  "gene_symbol": "IFT27",
  "gene_name": "Intraflagellar transport protein 27 homolog",
  "gene": "UniProtKB:Q9BW83"
}